sterol-dependent protein binding [GO:0070866] (molecular function) Relationships: is a type of GO:0005515 Sources: GOC:ecd Definition: Binding to a protein or protein complex in the presence of sterols.